{
  "term_label": "Unknown molecular function",
  "gene": "UniProtKB:Q8WUE5",
  "gene_symbol": "CT55",
  "gene_name": "Cancer_testis antigen 55",
  "term_id": "UNKNOWN:0001"
}